{
  "gene": "UniProtKB:Q8N0Y7",
  "gene_name": "Probable phosphoglycerate mutase 4",
  "term_label": "Unknown molecular function",
  "term_id": "UNKNOWN:0001",
  "gene_symbol": "PGAM4"
}